{
  "term_id": "GO:0075512",
  "gene_symbol": "SIGLEC1",
  "gene_name": "Sialoadhesin",
  "gene": "UniProtKB:Q9BZZ2",
  "term_label": "clathrin-dependent endocytosis of virus by host cell"
}